{
  "term_label": "ubiquitin-dependent protein catabolic process",
  "gene_symbol": "ENC1",
  "gene": "UniProtKB:O14682",
  "term_id": "GO:0006511",
  "gene_name": "Ectoderm-neural cortex protein 1"
}